{
  "gene_symbol": "UBAP2L",
  "gene": "UniProtKB:Q14157",
  "gene_name": "Ubiquitin-associated protein 2-like",
  "term_id": "GO:0061484",
  "term_label": "hematopoietic stem cell homeostasis"
}